{
  "term_id": "GO:0005615",
  "gene": "UniProtKB:P32881",
  "gene_name": "Interferon alpha-8",
  "term_label": "extracellular space",
  "gene_symbol": "IFNA8"
}